{
  "gene_name": "EGF-like repeat and discoidin I-like domain-containing protein 3",
  "gene": "UniProtKB:O43854",
  "term_id": "GO:0010811",
  "term_label": "positive regulation of cell-substrate adhesion",
  "gene_symbol": "EDIL3"
}